{
  "term_label": "Unknown biological process",
  "term_id": "UNKNOWN:0002",
  "gene_name": "Protein tyrosine phosphatase type IVA 2",
  "gene": "UniProtKB:Q12974",
  "gene_symbol": "PTP4A2"
}